{
  "term_label": "regulation of transcription by RNA polymerase II",
  "term_id": "GO:0006357",
  "gene": "UniProtKB:Q8N8G2",
  "gene_name": "Transcription cofactor vestigial-like protein 2",
  "gene_symbol": "VGLL2"
}